{
  "gene_name": "Apolipoprotein A-IV",
  "term_label": "cholesterol efflux",
  "gene": "UniProtKB:P06727",
  "gene_symbol": "APOA4",
  "term_id": "GO:0033344"
}